{
  "term_label": "proton transmembrane transport",
  "gene_symbol": "ATP4A",
  "gene_name": "Potassium-transporting ATPase alpha chain 1",
  "term_id": "GO:1902600",
  "gene": "UniProtKB:P20648"
}